ectodermal cell fate specification [GO:0001715] (biological process) Sources: GOC:go_curators Relationships: is a type of GO:0001708; is part of ectodermal cell fate commitment [GO:0001712] Regulation: regulated by regulation of ectodermal cell fate specification [GO:0042665]; negatively regulated by negative regulation of ectodermal cell fate specification [GO:0042666] Definition: The cell fate determination process that results in a cell becoming becomes capable of differentiating autonomously into an ectoderm cell in an environment that is neutral with respect to the developmental pathway; upon specification, the cell fate can be reversed. Also known as: ectoderm cell fate specification